{
  "term_id": "GO:0005743",
  "term_label": "mitochondrial inner membrane",
  "gene_symbol": "TIMM9",
  "gene": "UniProtKB:Q9Y5J7",
  "gene_name": "Mitochondrial import inner membrane translocase subunit Tim9"
}